{
  "gene": "UniProtKB:Q9NZA1",
  "term_label": "Unknown molecular function",
  "term_id": "UNKNOWN:0001",
  "gene_name": "Chloride intracellular channel protein 5",
  "gene_symbol": "CLIC5"
}